{
  "gene_name": "Hepatic triacylglycerol lipase",
  "gene": "UniProtKB:P11150",
  "term_id": "GO:0034375",
  "term_label": "high-density lipoprotein particle remodeling",
  "gene_symbol": "LIPC"
}